{
  "term_id": "GO:0001525",
  "gene_symbol": "PDGFB",
  "term_label": "angiogenesis",
  "gene_name": "Platelet-derived growth factor subunit B",
  "gene": "UniProtKB:P01127"
}